{
  "term_label": "Unknown biological process",
  "term_id": "UNKNOWN:0002",
  "gene_name": "Transmembrane protein 222",
  "gene": "UniProtKB:Q9H0R3",
  "gene_symbol": "TMEM222"
}